positive regulation of intracellular transport of viral material [GO:1901254] (biological process) Definition: Any process that activates or increases the frequency, rate or extent of intracellular transport of viral material. Also known as: activation of movement of virus within host cell, activation of viral egress, positive regulation of movement of virus within host cell, positive regulation of viral egress, up regulation of egress of virus within host cell, up regulation of movement of virus within host cell, up regulation of viral egress, up-regulation of egress of virus within host cell, up-regulation of movement of virus within host cell, up-regulation of viral egress, upregulation of egress of virus within host cell, upregulation of movement of virus within host cell, upregulation of viral egress, activation of egress of virus within host cell, positive regulation of egress of virus within host cell Sources: GOC:TermGenie, GOC:bf, GOC:jl Relationships: is a type of regulation of intracellular transport of viral material [GO:1901252]; is a type of GO:1903902; positively regulates intracellular transport of virus [GO:0075733]